{
  "term_id": "UNKNOWN:0002",
  "term_label": "Unknown biological process",
  "gene": "UniProtKB:E9PQ53",
  "gene_symbol": "NDUFC2-KCTD14",
  "gene_name": "NADH dehydrogenase [ubiquinone] 1 subunit C2, isoform 2"
}